establishment or maintenance of bipolar cell polarity regulating cell shape [GO:0061246] (biological process) Definition: Any cellular process that results in the specification, formation or maintenance of a bipolar intracellular organization or cell growth patterns that regulates the shaping of a cell. Subtypes: maintenance of bipolar cell polarity regulating cell shape [GO:0061305] Relationships: is a type of establishment or maintenance of bipolar cell polarity [GO:0061245]; is a type of establishment or maintenance of cell polarity regulating cell shape [GO:0071963] Sources: GOC:dph, GOC:vw Regulation: regulated by regulation of establishment or maintenance of bipolar cell polarity regulating cell shape [GO:2000100]; positively regulated by GO:2000247; negatively regulated by GO:2000750